{
  "term_label": "Unknown cellular component",
  "term_id": "UNKNOWN:0003",
  "gene_symbol": "ANKRD22",
  "gene_name": "Ankyrin repeat domain-containing protein 22",
  "gene": "UniProtKB:Q5VYY1"
}